JUN kinase kinase kinase activity [GO:0004706] (molecular function) Definition: Catalysis of the reaction: JNKK + ATP = JNKK phosphate + ADP. This reaction is the phosphorylation and activation of JUN kinase kinases (JNKKs). Relationships: is a type of GO:0004709 Also known as: JNKKK, JNK kinase kinase activity Sources: GOC:bf